{
  "gene_name": "Leucine-rich repeat and IQ domain-containing protein 3",
  "gene_symbol": "LRRIQ3",
  "term_id": "UNKNOWN:0002",
  "term_label": "Unknown biological process",
  "gene": "UniProtKB:A6PVS8"
}